{
  "gene_name": "Dedicator of cytokinesis protein 10",
  "gene": "UniProtKB:Q96BY6",
  "term_label": "dendritic spine morphogenesis",
  "gene_symbol": "DOCK10",
  "term_id": "GO:0060997"
}